{
  "gene": "UniProtKB:P48058",
  "gene_name": "Glutamate receptor 4",
  "term_id": "GO:0032281",
  "term_label": "AMPA glutamate receptor complex",
  "gene_symbol": "GRIA4"
}